regulation of Fas signaling pathway [GO:1902044] (biological process) Definition: Any process that modulates the frequency, rate or extent of Fas signaling pathway. References: PMID:17245429 Sources: GOC:TermGenie Also known as: regulation of Apo-1 signaling pathway, regulation of CD95 signaling pathway, regulation of Fas receptor signaling pathway, regulation of FasR signaling pathway, regulation of FAS ligand-Fas signaling pathway, regulation of Fas-FasL signaling pathway, regulation of FasL signaling pathway Relationships: is a type of regulation of signal transduction [GO:0009966]; regulates Fas signaling pathway [GO:0036337] Subtypes: negative regulation of Fas signaling pathway [GO:1902045], GO:1902046